{
  "gene_symbol": "DIS3",
  "term_label": "nuclear mRNA surveillance of mRNA 3'-end processing",
  "term_id": "GO:0071031",
  "gene": "UniProtKB:Q9Y2L1",
  "gene_name": "Exosome complex exonuclease RRP44"
}